{
  "term_label": "synaptic membrane",
  "gene_symbol": "ADAM10",
  "gene_name": "Disintegrin and metalloproteinase domain-containing protein 10",
  "gene": "UniProtKB:O14672",
  "term_id": "GO:0097060"
}